{
  "term_id": "GO:0002767",
  "gene_name": "Leukocyte-associated immunoglobulin-like receptor 1",
  "gene_symbol": "LAIR1",
  "term_label": "immune response-inhibiting cell surface receptor signaling pathway",
  "gene": "UniProtKB:Q6GTX8"
}